{
  "gene": "UniProtKB:Q9NS91",
  "gene_symbol": "RAD18",
  "term_label": "Unknown molecular function",
  "gene_name": "E3 ubiquitin-protein ligase RAD18",
  "term_id": "UNKNOWN:0001"
}